{
  "term_label": "RNA polymerase II cis-regulatory region sequence-specific DNA binding",
  "gene_name": "Krueppel-like factor 11",
  "gene": "UniProtKB:O14901",
  "term_id": "GO:0000978",
  "gene_symbol": "KLF11"
}